{
  "gene": "UniProtKB:P68106",
  "gene_name": "Peptidyl-prolyl cis-trans isomerase FKBP1B",
  "term_label": "sarcoplasmic reticulum membrane",
  "term_id": "GO:0033017",
  "gene_symbol": "FKBP1B"
}